histone deacetylase binding [GO:0042826] (molecular function) Definition: Binding to histone deacetylase. Sources: GOC:jl Relationships: is a type of enzyme binding [GO:0019899]